host cell extracellular matrix binding [GO:0046810] (molecular function) References: PMID:7996163 Relationships: is a type of GO:0050840 Definition: Binding to the extracellular matrix of a host cell.